{
  "gene": "UniProtKB:Q7Z5P9",
  "gene_name": "Mucin-19",
  "term_label": "Unknown cellular component",
  "gene_symbol": "MUC19",
  "term_id": "UNKNOWN:0003"
}